pronephric duct morphogenesis [GO:0039023] (biological process) Sources: GOC:mtg_kidney_jan10, XAO:0000063, ZFA:0000150 Definition: The process in which the anatomical structures of the pronephric duct are generated and organized. The pronephric duct collects the filtrate from the pronephric tubules and opens to the exterior of the kidney. Relationships: is a type of nephric duct morphogenesis [GO:0072178]; is part of GO:0039022; BFO_0000050 pronephros morphogenesis [GO:0072114]